icosahedral viral capsid [GO:0019030] (cellular component) Also known as: quasispherical viral capsid Relationships: is a type of viral capsid [GO:0019028] Definition: The protein coat that surrounds the infective nucleic acid in some virus particles; the subunits are arranged to form an icosahedron, a solid with 20 faces and 12 vertices. Icosahedral capsids have 12 pentamers plus 10(T-1) hexamers, where T is the triangulation number. Tobacco satellite necrosis virus has such a capsid structure. Sources: GOC:bm, ISBN:0198506732, ISBN:071673706X, VZ:885, Wikipedia:Capsid Subtypes: T=1 icosahedral viral capsid [GO:0039615], T=2 icosahedral viral capsid [GO:0039616], T=3 icosahedral viral capsid [GO:0039617], T=pseudo3 icosahedral viral capsid [GO:0039618], T=4 icosahedral viral capsid [GO:0039619], T=7 icosahedral viral capsid [GO:0039620], GO:0039621, T=16 icosahedral viral capsid [GO:0039622], T=25 icosahedral viral capsid [GO:0039623], T=147 icosahedral capsid [GO:0039627], T=169 icosahedral viral capsid [GO:0039628], GO:0039629, T=9 icosahedral viral capsid [GO:0160168], T=21/pseudo21 icosahedral capsid [GO:0160169], T=27/pseudo27 icosahedral capsid [GO:0160170], T=28 icosahedral capsid [GO:0160171], T=31/pseudo31 icosahedral capsid [GO:0160172]